{
  "gene_symbol": "KBTBD13",
  "term_label": "Unknown cellular component",
  "term_id": "UNKNOWN:0003",
  "gene_name": "Kelch repeat and BTB domain-containing protein 13",
  "gene": "UniProtKB:C9JR72"
}